{
  "gene_name": "Zinc finger and SCAN domain-containing protein 2",
  "gene_symbol": "ZSCAN2",
  "gene": "UniProtKB:Q7Z7L9",
  "term_id": "GO:0006357",
  "term_label": "regulation of transcription by RNA polymerase II"
}